{
  "gene_name": "SWI_SNF-related matrix-associated actin-dependent regulator of chromatin subfamily A member 5",
  "gene": "UniProtKB:O60264",
  "term_label": "nucleus",
  "gene_symbol": "SMARCA5",
  "term_id": "GO:0005634"
}